{
  "term_id": "GO:0043161",
  "gene_symbol": "SIAH1",
  "gene": "UniProtKB:Q8IUQ4",
  "term_label": "proteasome-mediated ubiquitin-dependent protein catabolic process",
  "gene_name": "E3 ubiquitin-protein ligase SIAH1"
}